{
  "term_label": "integrin-mediated signaling pathway",
  "gene": "UniProtKB:O75326",
  "gene_name": "Semaphorin-7A",
  "gene_symbol": "SEMA7A",
  "term_id": "GO:0007229"
}